{
  "term_label": "protein urmylation",
  "gene": "UniProtKB:Q9BTM9",
  "gene_symbol": "URM1",
  "gene_name": "Ubiquitin-related modifier 1",
  "term_id": "GO:0032447"
}